{
  "term_id": "GO:0019221",
  "gene_symbol": "IL7",
  "term_label": "cytokine-mediated signaling pathway",
  "gene_name": "Interleukin-7",
  "gene": "UniProtKB:P13232"
}